{
  "term_label": "DNA-binding transcription factor activity, RNA polymerase II-specific",
  "gene_name": "Class A basic helix-loop-helix protein 15",
  "gene_symbol": "BHLHA15",
  "term_id": "GO:0000981",
  "gene": "UniProtKB:Q7RTS1"
}